hormone metabolic process [GO:0042445] (biological process) Sources: GOC:jl Relationships: is a type of metabolic process [GO:0008152]; is a type of regulation of hormone levels [GO:0010817] Subtypes: juvenile hormone metabolic process [GO:0006716], C21-steroid hormone metabolic process [GO:0008207], androgen metabolic process [GO:0008209], estrogen metabolic process [GO:0008210], mineralocorticoid metabolic process [GO:0008212], cytokinin metabolic process [GO:0009690], GO:0009850, brassinosteroid metabolic process [GO:0016131], peptide hormone processing [GO:0016486], GO:0030186, GO:0042403, hormone biosynthetic process [GO:0042446], GO:0042447, retinol metabolic process [GO:0042572], retinoic acid metabolic process [GO:0042573], pheromone metabolic process [GO:0042810], ecdysteroid metabolic process [GO:0045455], prolactin metabolic process [GO:0120122] Definition: The chemical reactions and pathways involving any hormone, naturally occurring substances secreted by specialized cells that affects the metabolism or behavior of other cells possessing functional receptors for the hormone. Regulation: regulated by regulation of hormone metabolic process [GO:0032350]; negatively regulated by negative regulation of hormone metabolic process [GO:0032351]; positively regulated by positive regulation of hormone metabolic process [GO:0032352] Also known as: hormone metabolism, cellular hormone metabolic process